{
  "term_id": "GO:0005549",
  "gene_symbol": "OR4E1",
  "gene": "UniProtKB:P0C645",
  "gene_name": "Olfactory receptor 4E1",
  "term_label": "odorant binding"
}